{
  "gene_symbol": "AGPAT2",
  "term_label": "endoplasmic reticulum",
  "term_id": "GO:0005783",
  "gene_name": "1-acyl-sn-glycerol-3-phosphate acyltransferase beta",
  "gene": "UniProtKB:O15120"
}